{
  "term_label": "catalytic step 2 spliceosome",
  "gene_name": "Heterogeneous nuclear ribonucleoproteins A2_B1",
  "term_id": "GO:0071013",
  "gene": "UniProtKB:P22626",
  "gene_symbol": "HNRNPA2B1"
}